{
  "gene": "UniProtKB:Q9NVX2",
  "term_label": "Unknown molecular function",
  "gene_name": "Notchless protein homolog 1",
  "gene_symbol": "NLE1",
  "term_id": "UNKNOWN:0001"
}